ferulate biosynthetic process [GO:0033495] (biological process) Definition: The chemical reactions and pathways resulting in the formation of ferulate, (2E)-3-(4-hydroxy-3-methoxyphenyl)prop-2-enoate. Sources: GOC:mah Also known as: ferulate anabolism, ferulate biosynthesis, ferulate formation, ferulate synthesis Relationships: is a type of ferulate metabolic process [GO:0033494]; is a type of phenol-containing compound biosynthetic process [GO:0046189]; is a type of monocarboxylic acid biosynthetic process [GO:0072330]; is a type of olefinic compound biosynthetic process [GO:0120255]; is a type of ether biosynthetic process [GO:1901503]